{
  "gene": "UniProtKB:Q9UIL4",
  "term_id": "GO:0005874",
  "term_label": "microtubule",
  "gene_name": "Kinesin-like protein KIF25",
  "gene_symbol": "KIF25"
}